{
  "term_id": "GO:0006289",
  "term_label": "nucleotide-excision repair",
  "gene": "UniProtKB:P15927",
  "gene_symbol": "RPA2",
  "gene_name": "Replication protein A 32 kDa subunit"
}